{
  "gene_name": "mRNA decay activator protein ZFP36L2",
  "term_label": "cytosol",
  "gene_symbol": "ZFP36L2",
  "term_id": "GO:0005829",
  "gene": "UniProtKB:P47974"
}